mRNA destabilization [GO:0061157] (biological process) Subtypes: nuclear-transcribed mRNA catabolic process, deadenylation-dependent decay [GO:0000288], miRNA-mediated gene silencing by mRNA destabilization [GO:0035279], 3'-UTR-mediated mRNA destabilization [GO:0061158], polyadenylation-dependent mRNA catabolic process [GO:0071047], siRNA-mediated gene silencing by mRNA destabilization [GO:0090625], GO:0140991, transposable element silencing by mRNA destabilization [GO:0141008], polyuridylation-dependent mRNA catabolic process [GO:1990074] Sources: GOC:dph, GOC:jh Relationships: is a type of negative regulation of gene expression [GO:0010629]; is a type of GO:0043488; is a type of RNA destabilization [GO:0050779]; is a type of GO:0061014 Definition: Any process that decreases the stability of an mRNA molecule, making it more vulnerable to degradative processes. Messenger RNA is the intermediate molecule between DNA and protein. It includes UTR and coding sequences. It does not contain introns.